positive regulation of flavonoid biosynthetic process [GO:0009963] (biological process) Definition: Any process that activates or increases the frequency, rate or extent of the chemical reactions and pathways resulting in the formation of flavonoids. Sources: GOC:tb Also known as: positive regulation of flavonoid anabolism, positive regulation of flavonoid biosynthesis, positive regulation of flavonoid formation, positive regulation of flavonoid synthesis, up regulation of flavonoid biosynthetic process, up-regulation of flavonoid biosynthetic process, upregulation of flavonoid biosynthetic process, activation of flavonoid biosynthetic process, stimulation of flavonoid biosynthetic process Relationships: is a type of positive regulation of biosynthetic process [GO:0009891]; is a type of regulation of flavonoid biosynthetic process [GO:0009962]; positively regulates flavonoid biosynthetic process [GO:0009813] Subtypes: positive regulation of anthocyanin biosynthetic process [GO:0031542], positive regulation of flavonol biosynthetic process [GO:1900386]